{
  "gene": "UniProtKB:Q6IAA8",
  "term_id": "GO:0060090",
  "gene_name": "Ragulator complex protein LAMTOR1",
  "term_label": "molecular adaptor activity",
  "gene_symbol": "LAMTOR1"
}